{
  "gene": "UniProtKB:P15248",
  "term_id": "UNKNOWN:0002",
  "term_label": "Unknown biological process",
  "gene_symbol": "IL9",
  "gene_name": "Interleukin-9"
}